toll-like receptor 10 signaling pathway [GO:0034166] (biological process) Relationships: is a type of cell surface toll-like receptor signaling pathway [GO:0140895] Definition: The series of molecular signals initiated by a ligand binding to toll-like receptor 10. Also known as: TLR10 signaling pathway, toll-like receptor 10 signalling pathway References: PMID:16551253, PMID:17328678 Sources: GOC:add Regulation: regulated by regulation of toll-like receptor 10 signaling pathway [GO:0034167]; negatively regulated by negative regulation of toll-like receptor 10 signaling pathway [GO:0034168]; positively regulated by positive regulation of toll-like receptor 10 signaling pathway [GO:0034169]